epithelial cell migration involved in metanephric nephron tubule morphogenesis [GO:0072290] (biological process) Subtypes: GO:0072291, epithelial cell migration involved in metanephric proximal tubule morphogenesis [GO:0072292] Sources: GOC:mtg_kidney_jan10 Relationships: is a type of cell migration involved in metanephros development [GO:0035788]; is a type of GO:0072155; is part of metanephric nephron tubule morphogenesis [GO:0072282] Definition: The orderly movement of epithelial cells within a renal tubule that contributes to metanephric nephron tubule morphogenesis.